receptor localization to synapse [GO:0097120] (biological process) References: PMID:21525273 Sources: GOC:BHF, GOC:sjp Subtypes: GO:0098968, GO:0098969, postsynaptic neurotransmitter receptor diffusion trapping [GO:0098970], anterograde dendritic transport of neurotransmitter receptor complex [GO:0098971], neurotransmitter receptor localization to postsynaptic specialization membrane [GO:0099645], anterograde axonal transport of neurotransmitter receptor complex [GO:0140231], regulation of synaptic plasticity by receptor localization to synapse [GO:1900383] Relationships: is a type of GO:0051179 Definition: Any process in which a receptor is transported to, and/or maintained at the synapse, the junction between a nerve fiber of one neuron and another neuron or muscle fiber or glial cell. Also known as: receptor localisation to synapse Regulation: regulated by regulation of receptor localization to synapse [GO:1902683]; negatively regulated by GO:1902684; positively regulated by positive regulation of receptor localization to synapse [GO:1902685]